{
  "term_id": "GO:0036064",
  "term_label": "ciliary basal body",
  "gene_name": "Centrosomal protein CCDC61",
  "gene": "UniProtKB:Q9Y6R9",
  "gene_symbol": "CCDC61"
}